{
  "gene_name": "Transmembrane protein 225B",
  "gene_symbol": "TMEM225B",
  "term_id": "UNKNOWN:0003",
  "term_label": "Unknown cellular component",
  "gene": "UniProtKB:P0DP42"
}